{
  "gene_name": "Synaptotagmin-9",
  "gene": "UniProtKB:Q86SS6",
  "term_label": "SNARE binding",
  "term_id": "GO:0000149",
  "gene_symbol": "SYT9"
}